{
  "gene": "UniProtKB:A0A8V8TLL3",
  "term_id": "UNKNOWN:0001",
  "term_label": "Unknown molecular function",
  "gene_name": "Uncharacterized protein",
  "gene_symbol": "A0A8V8TLL3"
}